{
  "gene": "UniProtKB:Q96PC3",
  "term_label": "Unknown cellular component",
  "term_id": "UNKNOWN:0003",
  "gene_name": "AP-1 complex subunit sigma-3",
  "gene_symbol": "AP1S3"
}